{
  "term_label": "intracellular protein localization",
  "gene": "UniProtKB:Q8IWZ6",
  "term_id": "GO:0008104",
  "gene_name": "Bardet-Biedl syndrome 7 protein",
  "gene_symbol": "BBS7"
}